{
  "gene_name": "Pro-adrenomedullin",
  "gene_symbol": "ADM",
  "term_label": "hormone activity",
  "term_id": "GO:0005179",
  "gene": "UniProtKB:P35318"
}